positive regulation of terminal button organization [GO:1901614] (biological process) Also known as: positive regulation of bouton organization, positive regulation of presynaptic bouton organization, positive regulation of synaptic bouton organization, positive regulation of terminal bouton organization, positive regulation of terminal button organisation, up regulation of bouton organization, up regulation of presynaptic bouton organization, up regulation of synaptic bouton organization, up regulation of terminal bouton organization, up regulation of terminal button organisation, up regulation of terminal button organization, up-regulation of bouton organization, up-regulation of presynaptic bouton organization, up-regulation of synaptic bouton organization, up-regulation of terminal bouton organization, up-regulation of terminal button organisation, up-regulation of terminal button organization, upregulation of bouton organization, upregulation of presynaptic bouton organization, upregulation of synaptic bouton organization, upregulation of terminal bouton organization, upregulation of terminal button organisation, upregulation of terminal button organization, activation of bouton organization, activation of presynaptic bouton organization, activation of synaptic bouton organization, activation of terminal bouton organization, activation of terminal button organisation, activation of terminal button organization Definition: Any process that activates or increases the frequency, rate or extent of terminal button organization. Relationships: is a type of positive regulation of cellular component organization [GO:0051130]; is a type of GO:2000331; positively regulates GO:0072553 References: PMID:22426000 Sources: GOC:TermGenie